{
  "term_id": "UNKNOWN:0001",
  "gene": "UniProtKB:A8MV72",
  "term_label": "Unknown molecular function",
  "gene_symbol": "A8MV72",
  "gene_name": "Putative UPF0607 protein ENSP00000382826"
}